{
  "term_label": "cytokine activity",
  "gene_name": "Interleukin-31",
  "gene": "UniProtKB:Q6EBC2",
  "term_id": "GO:0005125",
  "gene_symbol": "IL31"
}